reversible differentiation [GO:0090677] (biological process) Sources: GOC:curators Definition: A phenotypic switching process where a cell reversibly differentiates and dedifferentiates from one cell type into another. Relationships: is a type of phenotypic switching [GO:0036166]